{
  "term_label": "Unknown biological process",
  "gene_symbol": "SORCS3",
  "gene": "UniProtKB:Q9UPU3",
  "gene_name": "VPS10 domain-containing receptor SorCS3",
  "term_id": "UNKNOWN:0002"
}